{
  "gene_symbol": "H2BC15",
  "term_id": "GO:0019731",
  "gene": "UniProtKB:Q99877",
  "term_label": "antibacterial humoral response",
  "gene_name": "Histone H2B type 1-N"
}